{
  "gene_name": "Probable bifunctional dTTP_UTP pyrophosphatase_methyltransferase protein",
  "gene": "UniProtKB:O95671",
  "term_label": "Unknown biological process",
  "term_id": "UNKNOWN:0002",
  "gene_symbol": "ASMTL"
}